{
  "gene_name": "Integrin alpha-8",
  "term_id": "GO:0008305",
  "gene_symbol": "ITGA8",
  "term_label": "integrin complex",
  "gene": "UniProtKB:P53708"
}